{
  "gene_symbol": "GPC2",
  "term_label": "cell migration",
  "gene": "UniProtKB:Q8N158",
  "term_id": "GO:0016477",
  "gene_name": "Glypican-2"
}